{
  "term_label": "G protein-coupled receptor activity",
  "term_id": "GO:0004930",
  "gene_name": "Hydroxycarboxylic acid receptor 1",
  "gene": "UniProtKB:Q9BXC0",
  "gene_symbol": "HCAR1"
}